{
  "gene": "UniProtKB:Q7Z7K6",
  "term_id": "GO:0005634",
  "gene_symbol": "CENPV",
  "term_label": "nucleus",
  "gene_name": "Centromere protein V"
}